gametophyte development [GO:0048229] (biological process) Relationships: is_a GO:0007275 Definition: The process whose specific outcome is the progression of the gametophyte over time, from its formation to the mature structure. The gametophyte is the gamete-producing individual or phase in the life cycle having alternation of generations. An example of this process is found in Arabidopsis thaliana. Also known as: gametogenesis Sources: GOC:jid, PO:0009004 Subtypes: embryo sac development [GO:0009553], pollen development [GO:0009555]